{
  "gene_name": "Tubulin beta chain",
  "term_label": "microtubule cytoskeleton organization",
  "gene_symbol": "TUBB",
  "term_id": "GO:0000226",
  "gene": "UniProtKB:P07437"
}